nucleokinesis involved in cell motility in cerebral cortex radial glia guided migration [GO:0021817] (biological process) Definition: The microtubule-mediated movement of the nucleus that is required for the movement of cells along radial glial fibers as a component of the process of cerebral cortex glial-mediated radial cell migration. References: PMID:12626695 Sources: GOC:cls, GOC:dgh, GOC:dph, GOC:jid, GOC:tb Relationships: is a type of nuclear migration along microtubule [GO:0030473]; is part of modulation of microtubule cytoskeleton involved in cerebral cortex radial glia guided migration [GO:0021815] Also known as: nucleokinesis involved in cell locomotion in cerebral cortex glial-mediated radial migration, nucleokinesis involved in cell locomotion in cerebral cortex radial glia guided migration